{
  "gene": "UniProtKB:Q9ULE3",
  "term_id": "GO:0042147",
  "gene_symbol": "DENND2A",
  "term_label": "retrograde transport, endosome to Golgi",
  "gene_name": "DENN domain-containing protein 2A"
}